{
  "gene_symbol": "FGF6",
  "term_id": "GO:0005737",
  "term_label": "cytoplasm",
  "gene_name": "Fibroblast growth factor 6",
  "gene": "UniProtKB:P10767"
}